{
  "term_id": "GO:0035615",
  "term_label": "clathrin adaptor activity",
  "gene_name": "AP-3 complex subunit mu-2",
  "gene": "UniProtKB:P53677",
  "gene_symbol": "AP3M2"
}